{
  "gene_name": "von Willebrand factor A domain-containing protein 5B1",
  "term_id": "UNKNOWN:0003",
  "gene_symbol": "VWA5B1",
  "term_label": "Unknown cellular component",
  "gene": "UniProtKB:Q5TIE3"
}